{
  "term_id": "UNKNOWN:0002",
  "gene": "UniProtKB:P62910",
  "gene_name": "Large ribosomal subunit protein eL32",
  "gene_symbol": "RPL32",
  "term_label": "Unknown biological process"
}